nitric oxide storage [GO:0035732] (biological process) Also known as: NO storage References: PMID:12871945 Sources: GOC:BHF Definition: The accumulation and maintenance in cells or tissues of nitric oxide (NO). Nitric oxide is stored in the form of dinitrosyl-iron complexes, which are stabilized, and possibly sequestered, by binding to glutathione S-transferase proteins. Relationships: is a type of GO:0051179; is part of GO:0033484